beta-N-acetylhexosaminidase activity [GO:0004563] (molecular function) Relationships: is a type of hexosaminidase activity [GO:0015929] Sources: EC:3.2.1.52 Definition: Catalysis of the hydrolysis of terminal non-reducing N-acetyl-D-hexosamine residues in N-acetyl-beta-D-hexosaminides. Subtypes: beta-N-acetylglucosaminidase activity [GO:0016231], beta-N-acetylgalactosaminidase activity [GO:0032428] Also known as: N-acetyl-beta-D-hexosaminidase activity, N-acetyl-beta-glucosaminidase activity, N-acetyl-beta-hexosaminidase activity, N-acetylhexosaminidase activity, beta-D-N-acetylhexosaminidase activity, beta-D-hexosaminidase activity, beta-N-acetyl-D-hexosaminidase activity, beta-N-acetyl-D-hexosaminide N-acetylhexosaminohydrolase activity, beta-acetylaminodeoxyhexosidase activity, beta-acetylhexosaminidinase activity, beta-hexosaminidase activity, hexosaminidase A